{
  "term_id": "GO:0008543",
  "gene_symbol": "FGF23",
  "gene": "UniProtKB:Q9GZV9",
  "term_label": "fibroblast growth factor receptor signaling pathway",
  "gene_name": "Fibroblast growth factor 23"
}